endonucleolytic cleavage in 5'-ETS of tricistronic rRNA transcript (SSU-rRNA, 5.8S rRNA, LSU-rRNA) [GO:0000480] (biological process) References: PMID:10690410, PMID:15282326 Sources: GOC:curators Definition: Endonucleolytic cleavage within the 5'-External Transcribed Spacer (ETS) of a tricistronic rRNA transcript that contains the Small Subunit (SSU) rRNA, the 5.8S rRNA, and the Large Subunit (LSU) rRNA in that order from 5' to 3' along the primary transcript. Endonucleolytic cleavage within the 5'-ETS of the pre-RNA is conserved as one of the early steps of rRNA processing in all eukaryotes, but the specific position of cleavage is variable. Relationships: is a type of endonucleolytic cleavage of tricistronic rRNA transcript (SSU-rRNA, 5.8S rRNA, LSU-rRNA) [GO:0000479]; is part of GO:0000462 Also known as: endonucleolytic cleavage at A-prime, endonucleolytic cleavage at A0